RNA uridine deletion [GO:0070710] (biological process) Also known as: RNA U deletion, RNA uridine excision Sources: GOC:cb, GOC:mah Definition: The modification of an RNA molecule by removal of a uridine nucleotide. Relationships: is a type of RNA nucleotide deletion [GO:0070706]